{
  "term_label": "nucleus",
  "gene": "UniProtKB:Q6AHZ1",
  "gene_symbol": "ZNF518A",
  "gene_name": "Zinc finger protein 518A",
  "term_id": "GO:0005634"
}